{
  "term_id": "UNKNOWN:0002",
  "term_label": "Unknown biological process",
  "gene_name": "Glutamine amidotransferase-like class 1 domain-containing protein 3, mitochondrial",
  "gene": "UniProtKB:P0DPI2",
  "gene_symbol": "GATD3"
}